{
  "gene_name": "Sodium-dependent lysophosphatidylcholine symporter 1",
  "term_label": "plasma membrane",
  "term_id": "GO:0005886",
  "gene_symbol": "MFSD2A",
  "gene": "UniProtKB:Q8NA29"
}